regulation of leukotriene production involved in inflammatory response [GO:0035490] (biological process) Subtypes: positive regulation of leukotriene production involved in inflammatory response [GO:0035491], GO:0035492 Sources: GOC:bf Relationships: is a type of regulation of multicellular organismal process [GO:0051239]; regulates leukotriene production involved in inflammatory response [GO:0002540] Definition: Any process that modulates the rate, frequency or extent of the synthesis or release of any leukotriene following a stimulus as part of an inflammatory response.